{
  "gene_symbol": "KRTAP2-2",
  "term_id": "UNKNOWN:0001",
  "gene_name": "Keratin-associated protein 2-2",
  "gene": "UniProtKB:Q9BYT5",
  "term_label": "Unknown molecular function"
}